{
  "gene": "UniProtKB:Q00013",
  "term_id": "UNKNOWN:0002",
  "term_label": "Unknown biological process",
  "gene_name": "55 kDa erythrocyte membrane protein",
  "gene_symbol": "MPP1"
}